{
  "term_label": "translesion synthesis",
  "gene_name": "DNA-directed primase_polymerase protein",
  "term_id": "GO:0019985",
  "gene": "UniProtKB:Q96LW4",
  "gene_symbol": "PRIMPOL"
}